{
  "gene": "UniProtKB:A6NEY8",
  "term_label": "Unknown cellular component",
  "gene_symbol": "PRORSD1P",
  "gene_name": "Putative prolyl-tRNA synthetase associated domain-containing protein 1",
  "term_id": "UNKNOWN:0003"
}